guanosine catabolic process [GO:0046115] (BP) Definition: The chemical reactions and pathways resulting in the breakdown of guanine, guanine riboside, a nucleoside with a wide species distribution. Also known as: guanosine breakdown, guanosine catabolism, guanosine degradation, guanosine phosphorolysis Sources: GOC:go_curators Relationships: is a type of guanosine metabolic process [GO:0008617]; is a type of GO:1901069